{
  "gene_symbol": "PLXND1",
  "term_label": "synapse assembly",
  "term_id": "GO:0007416",
  "gene_name": "Plexin-D1",
  "gene": "UniProtKB:Q9Y4D7"
}